{
  "gene_name": "Beta-crystallin B2",
  "term_label": "Unknown cellular component",
  "term_id": "UNKNOWN:0003",
  "gene": "UniProtKB:P43320",
  "gene_symbol": "CRYBB2"
}